prolactin-releasing peptide receptor binding [GO:0031861] (molecular function) Also known as: prolactin-releasing peptide receptor ligand Relationships: is a type of neuropeptide receptor binding [GO:0071855] Sources: GOC:mah, GOC:nln Definition: Binding to a prolactin-releasing peptide receptor.